interleukin-1 type II receptor antagonist activity [GO:0045353] (molecular function) Relationships: is a type of interleukin-1 receptor antagonist activity [GO:0005152] Also known as: IL-1ra type II Definition: Blocks the binding of interleukin-1 to interleukin-1 type II receptors. Sources: GOC:ebc